{
  "gene_name": "Leucine-rich repeat and IQ domain-containing protein 3",
  "term_id": "UNKNOWN:0003",
  "gene_symbol": "LRRIQ3",
  "gene": "UniProtKB:A6PVS8",
  "term_label": "Unknown cellular component"
}